{
  "gene_name": "Testis-specific gene 10 protein",
  "term_label": "motile cilium",
  "gene": "UniProtKB:Q9BZW7",
  "term_id": "GO:0031514",
  "gene_symbol": "TSGA10"
}